{
  "term_id": "UNKNOWN:0002",
  "term_label": "Unknown biological process",
  "gene": "UniProtKB:A0A0G2JLE6",
  "gene_symbol": "KRTAP4-8",
  "gene_name": "HCG2042992"
}